{
  "gene": "UniProtKB:Q9BVC4",
  "term_label": "Unknown molecular function",
  "gene_name": "Target of rapamycin complex subunit LST8",
  "gene_symbol": "MLST8",
  "term_id": "UNKNOWN:0001"
}